{
  "term_label": "Unknown molecular function",
  "gene_name": "Nck-associated protein 1",
  "term_id": "UNKNOWN:0001",
  "gene": "UniProtKB:Q9Y2A7",
  "gene_symbol": "NCKAP1"
}